{
  "term_label": "Unknown biological process",
  "term_id": "UNKNOWN:0002",
  "gene_symbol": "PRADC1",
  "gene": "UniProtKB:Q9BSG0",
  "gene_name": "Protease-associated domain-containing protein 1"
}